{
  "gene_symbol": "AK3",
  "gene": "UniProtKB:Q9UIJ7",
  "gene_name": "GTP:AMP phosphotransferase AK3, mitochondrial",
  "term_label": "nucleoside triphosphate biosynthetic process",
  "term_id": "GO:0009142"
}